{
  "term_id": "UNKNOWN:0002",
  "gene_name": "Monoglyceride lipase",
  "gene": "UniProtKB:Q99685",
  "gene_symbol": "MGLL",
  "term_label": "Unknown biological process"
}